{
  "term_label": "plasma membrane",
  "gene_name": "Transmembrane protease serine 7",
  "gene": "UniProtKB:Q7RTY8",
  "gene_symbol": "TMPRSS7",
  "term_id": "GO:0005886"
}